{
  "gene_name": "Centriole, cilia and spindle-associated protein",
  "gene": "UniProtKB:Q6IQ19",
  "gene_symbol": "CCSAP",
  "term_id": "GO:0036064",
  "term_label": "ciliary basal body"
}